cellular response to triacyl bacterial lipopeptide [GO:0071727] (biological process) Relationships: is a type of cellular response to bacterial lipopeptide [GO:0071221]; is a type of response to triacyl bacterial lipopeptide [GO:0071725] Also known as: cellular response to triacylated bacterial lipoprotein Definition: Any process that results in a change in state or activity of a cell (in terms of movement, secretion, enzyme production, gene expression, etc.) as a result of a triacylated bacterial lipopeptide stimulus. References: PMID:12077222, PMID:12524386, PMID:2757794 Sources: GOC:add Note: Note that bacterial lipopeptides are derived from bacterial lipoproteins, but the two terms are sometimes used interchangeably in the literature.